{
  "term_id": "GO:0005096",
  "gene_name": "Ras_Rap GTPase-activating protein SynGAP",
  "term_label": "GTPase activator activity",
  "gene_symbol": "SYNGAP1",
  "gene": "UniProtKB:Q96PV0"
}